{
  "gene_symbol": "CIAO2B",
  "gene_name": "Cytosolic iron-sulfur assembly component 2B",
  "term_label": "cytosolic [4Fe-4S] assembly targeting complex",
  "gene": "UniProtKB:Q9Y3D0",
  "term_id": "GO:0097361"
}